{
  "gene": "UniProtKB:Q9H9Z2",
  "gene_symbol": "LIN28A",
  "gene_name": "Protein lin-28 homolog A",
  "term_label": "mRNA binding",
  "term_id": "GO:0003729"
}